{
  "term_label": "mRNA binding",
  "gene": "UniProtKB:Q9BY44",
  "gene_symbol": "EIF2A",
  "term_id": "GO:0003729",
  "gene_name": "Eukaryotic translation initiation factor 2A"
}